{
  "gene": "UniProtKB:Q9BQK8",
  "term_id": "GO:0009062",
  "term_label": "fatty acid catabolic process",
  "gene_symbol": "LPIN3",
  "gene_name": "Phosphatidate phosphatase LPIN3"
}